{
  "term_label": "Unknown biological process",
  "term_id": "UNKNOWN:0002",
  "gene_name": "Protein FAM98C",
  "gene": "UniProtKB:Q17RN3",
  "gene_symbol": "FAM98C"
}